{
  "term_id": "UNKNOWN:0001",
  "gene": "UniProtKB:Q9BT67",
  "gene_name": "NEDD4 family-interacting protein 1",
  "gene_symbol": "NDFIP1",
  "term_label": "Unknown molecular function"
}